pyrimidine deoxyribonucleoside diphosphate catabolic process [GO:0009198] (biological process) Sources: GOC:go_curators, ISBN:0198506732 Definition: The chemical reactions and pathways resulting in the breakdown of pyrimidine deoxynucleoside diphosphate, a compound consisting of a pyrimidine base linked to a deoxyribose sugar esterified with diphosphate on the sugar. Relationships: is a type of pyrimidine nucleoside diphosphate catabolic process [GO:0009140]; is a type of GO:0009192; is a type of pyrimidine deoxyribonucleoside diphosphate metabolic process [GO:0009196] Subtypes: dTDP catabolic process [GO:0006246], dCDP catabolic process [GO:0006251], GO:0006257 Also known as: pyrimidine deoxyribonucleoside diphosphate breakdown, pyrimidine deoxyribonucleoside diphosphate catabolism, pyrimidine deoxyribonucleoside diphosphate degradation